{
  "gene": "UniProtKB:Q8WUH6",
  "gene_name": "Transmembrane protein 263",
  "term_label": "Unknown molecular function",
  "gene_symbol": "TMEM263",
  "term_id": "UNKNOWN:0001"
}